vomifoliol 4'-dehydrogenase activity [GO:0050396] (MF) Definition: Catalysis of the reaction: (6S,9R)-6-hydroxy-3-oxo-alpha-ionol + NAD+ = (6S)-6-hydroxy-3-oxo-alpha-ionone + H+ + NADH. Sources: EC:1.1.1.221, RHEA:22804 Also known as: vomifoliol:NAD+ 4'-oxidoreductase activity Relationships: is a type of oxidoreductase activity, acting on the CH-OH group of donors, NAD or NADP as acceptor [GO:0016616]